{
  "term_id": "UNKNOWN:0001",
  "gene_name": "T cell receptor alpha variable 26-2",
  "gene_symbol": "TRAV26-2",
  "term_label": "Unknown molecular function",
  "gene": "UniProtKB:A0A0B4J265"
}